sperm DNA decondensation [GO:0035041] (BP) Also known as: sperm chromatin decondensation Relationships: is a type of GO:0006325; is part of GO:0035039 References: PMID:11735001, PMID:23352575 Sources: GOC:bf Definition: Unwinding of the condensed nuclear chromatin of an inactive male pronucleus after fertilization.